{
  "gene_name": "Transcription factor SOX-2",
  "gene_symbol": "SOX2",
  "gene": "UniProtKB:P48431",
  "term_label": "DNA-binding transcription activator activity, RNA polymerase II-specific",
  "term_id": "GO:0001228"
}